voltage-gated sodium channel activity involved in AV node cell action potential [GO:0086060] (molecular function) Sources: GOC:BHF, GOC:mtg_cardiac_conduct_nov11 Also known as: voltage-gated sodium channel activity involved in AV node cardiac muscle cell action potential, voltage-gated sodium channel activity involved in atrioventricular node cardiac muscle cell action potential Definition: Enables the transmembrane transfer of a sodium ion by a voltage-gated channel through the plasma membrane of an AV node cardiac muscle cell contributing to the depolarization phase of an action potential. A voltage-gated channel is a channel whose open state is dependent on the voltage across the membrane in which it is embedded. Relationships: is_a voltage-gated sodium channel activity involved in cardiac muscle cell action potential [GO:0086006]; is part of GO:0086045